{
  "term_label": "interphase microtubule organizing center",
  "gene_name": "Cytoplasmic dynein 2 intermediate chain 1",
  "gene": "UniProtKB:Q8WVS4",
  "term_id": "GO:0031021",
  "gene_symbol": "DYNC2I1"
}